{
  "gene_name": "Fibrous sheath CABYR-binding protein",
  "gene_symbol": "FSCB",
  "gene": "UniProtKB:Q5H9T9",
  "term_id": "GO:0005509",
  "term_label": "calcium ion binding"
}